{
  "term_label": "Unknown molecular function",
  "term_id": "UNKNOWN:0001",
  "gene_symbol": "TMEM119",
  "gene_name": "Transmembrane protein 119",
  "gene": "UniProtKB:Q4V9L6"
}